{
  "gene_name": "Stalled ribosome sensor GCN1",
  "gene": "UniProtKB:Q92616",
  "term_id": "GO:0006417",
  "gene_symbol": "GCN1",
  "term_label": "regulation of translation"
}